{
  "gene": "UniProtKB:Q8TD84",
  "gene_name": "Cell adhesion molecule DSCAML1",
  "gene_symbol": "DSCAML1",
  "term_label": "cell-cell adhesion mediator activity",
  "term_id": "GO:0098632"
}